positive regulation of isoprene biosynthetic process [GO:1900949] (biological process) Sources: GOC:TermGenie, GOC:mengo_curators Definition: Any process that activates or increases the frequency, rate or extent of isoprene biosynthetic process. Also known as: positive regulation of 2-methyl-1,3-butadiene biosynthesis, positive regulation of 2-methyl-1,3-butadiene biosynthetic process, positive regulation of hemiterpene biosynthesis, positive regulation of hemiterpene biosynthetic process, up regulation of 2-methyl-1,3-butadiene biosynthesis, up regulation of 2-methyl-1,3-butadiene biosynthetic process, up regulation of hemiterpene biosynthesis, up regulation of hemiterpene biosynthetic process, up regulation of isoprene biosynthetic process, up-regulation of 2-methyl-1,3-butadiene biosynthesis, up-regulation of 2-methyl-1,3-butadiene biosynthetic process, up-regulation of hemiterpene biosynthesis, up-regulation of hemiterpene biosynthetic process, up-regulation of isoprene biosynthetic process, upregulation of 2-methyl-1,3-butadiene biosynthesis, upregulation of 2-methyl-1,3-butadiene biosynthetic process, upregulation of hemiterpene biosynthesis, upregulation of hemiterpene biosynthetic process, upregulation of isoprene biosynthetic process, activation of 2-methyl-1,3-butadiene biosynthesis, activation of 2-methyl-1,3-butadiene biosynthetic process, activation of hemiterpene biosynthesis, activation of hemiterpene biosynthetic process, activation of isoprene biosynthetic process Relationships: is a type of positive regulation of lipid biosynthetic process [GO:0046889]; is_a positive regulation of olefin biosynthetic process [GO:1900913]; is a type of regulation of isoprene biosynthetic process [GO:1900947]; positively regulates isoprene biosynthetic process [GO:0043612]